{
  "gene_symbol": "ESRRA",
  "gene_name": "Steroid hormone receptor ERR1",
  "term_label": "estrogen response element binding",
  "term_id": "GO:0034056",
  "gene": "UniProtKB:P11474"
}